{
  "gene": "UniProtKB:Q8TCU3",
  "term_label": "L-amino acid transmembrane transporter activity",
  "gene_name": "Solute carrier family 7 member 13",
  "term_id": "GO:0015179",
  "gene_symbol": "SLC7A13"
}